{
  "gene_name": "Adenosine receptor A3",
  "term_id": "GO:0005886",
  "gene": "UniProtKB:P0DMS8",
  "gene_symbol": "ADORA3",
  "term_label": "plasma membrane"
}